{
  "term_id": "GO:0004984",
  "gene_symbol": "OR1D5",
  "gene": "UniProtKB:P58170",
  "gene_name": "Olfactory receptor 1D5",
  "term_label": "olfactory receptor activity"
}